{
  "gene_symbol": "CSPP1",
  "term_label": "positive regulation of cytokinesis",
  "gene_name": "Centrosome and spindle pole-associated protein 1",
  "gene": "UniProtKB:Q1MSJ5",
  "term_id": "GO:0032467"
}